{
  "gene_name": "Metabotropic glutamate receptor 8",
  "term_label": "regulation of synaptic transmission, glutamatergic",
  "gene_symbol": "GRM8",
  "gene": "UniProtKB:O00222",
  "term_id": "GO:0051966"
}